{
  "gene_name": "Tubulin alpha-1C chain",
  "gene_symbol": "TUBA1C",
  "term_id": "GO:0000278",
  "gene": "UniProtKB:Q9BQE3",
  "term_label": "mitotic cell cycle"
}